{
  "term_label": "interleukin-3-mediated signaling pathway",
  "gene": "UniProtKB:P08700",
  "gene_symbol": "IL3",
  "term_id": "GO:0038156",
  "gene_name": "Interleukin-3"
}